{
  "term_label": "cortical actin cytoskeleton organization",
  "gene_symbol": "ROCK1",
  "term_id": "GO:0030866",
  "gene_name": "Rho-associated protein kinase 1",
  "gene": "UniProtKB:Q13464"
}